positive regulation of L-arginine import across plasma membrane [GO:1905589] (biological process) Also known as: positive regulation of L-arginine import, activation of L-arginine uptake, positive regulation of L-arginine import into cell, positive regulation of L-arginine uptake, up regulation of L-arginine import, up regulation of L-arginine uptake, up-regulation of L-arginine import, up-regulation of L-arginine import into cell, up-regulation of L-arginine uptake, upregulation of L-arginine import, upregulation of L-arginine import into cell, upregulation of L-arginine uptake, activation of L-arginine import, activation of L-arginine import across plasma membrane, activation of L-arginine import into cell References: PMID:14718525 Sources: GOC:TermGenie, GO_REF:0000058 Definition: Any process that activates or increases the frequency, rate or extent of L-arginine import across plasma membrane. Relationships: is a type of GO:0032892; is a type of positive regulation of transmembrane transport [GO:0034764]; is a type of positive regulation of amino acid transport [GO:0051957]; is a type of GO:1905541; positively regulates L-arginine import across plasma membrane [GO:0097638]